{
  "term_label": "Unknown biological process",
  "gene_symbol": "YDJC",
  "gene": "UniProtKB:A8MPS7",
  "term_id": "UNKNOWN:0002",
  "gene_name": "Carbohydrate deacetylase"
}